{
  "term_id": "GO:0016567",
  "gene_symbol": "DTX3",
  "term_label": "protein ubiquitination",
  "gene": "UniProtKB:Q8N9I9",
  "gene_name": "Probable E3 ubiquitin-protein ligase DTX3"
}